{
  "term_id": "UNKNOWN:0002",
  "term_label": "Unknown biological process",
  "gene_name": "Putative uncharacterized protein encoded by LINC00303",
  "gene_symbol": "LINC00303",
  "gene": "UniProtKB:Q3SY05"
}